positive regulation of natural killer cell apoptotic process [GO:0070249] (biological process) Definition: Any process that activates or increases the frequency, rate or extent of natural killer cell death by apoptotic process. Sources: GOC:add, GOC:mtg_apoptosis, ISBN:0781765196 Relationships: is_a positive regulation of lymphocyte apoptotic process [GO:0070230]; is a type of regulation of natural killer cell apoptotic process [GO:0070247]; positively regulates natural killer cell apoptotic process [GO:0070246] Also known as: positive regulation of NK cell apoptosis, up regulation of natural killer cell apoptosis, up-regulation of natural killer cell apoptosis, upregulation of natural killer cell apoptosis, activation of natural killer cell apoptosis, positive regulation of natural killer cell apoptosis, stimulation of natural killer cell apoptosis